{
  "gene": "UniProtKB:Q9HBA0",
  "term_label": "actin filament organization",
  "gene_name": "Transient receptor potential cation channel subfamily V member 4",
  "gene_symbol": "TRPV4",
  "term_id": "GO:0007015"
}